{
  "term_label": "Unknown biological process",
  "gene_symbol": "DCST2",
  "gene": "UniProtKB:Q5T1A1",
  "term_id": "UNKNOWN:0002",
  "gene_name": "DC-STAMP domain-containing protein 2"
}